{
  "term_id": "GO:0005737",
  "gene_name": "von Willebrand factor C and EGF domain-containing protein",
  "term_label": "cytoplasm",
  "gene": "UniProtKB:Q96DN2",
  "gene_symbol": "VWCE"
}